{
  "gene": "UniProtKB:Q9HCJ6",
  "gene_name": "Synaptic vesicle membrane protein VAT-1 homolog-like",
  "term_label": "Unknown molecular function",
  "gene_symbol": "VAT1L",
  "term_id": "UNKNOWN:0001"
}